{
  "gene_name": "Forkhead box protein D2",
  "gene_symbol": "FOXD2",
  "term_label": "Unknown cellular component",
  "gene": "UniProtKB:O60548",
  "term_id": "UNKNOWN:0003"
}